meiotic cohesin complex [GO:0030893] (cellular component) References: PMID:12750522 Sources: GOC:mah Definition: A cohesin complex that mediates sister chromatid cohesion during meiosis; has a subunit composition distinct from that of the mitotic cohesin complex. Relationships: is a type of GO:0008278 Also known as: nuclear meiotic cohesin complex